{
  "term_id": "GO:0008486",
  "gene_name": "Diphosphoinositol polyphosphate phosphohydrolase NUDT4B",
  "gene": "UniProtKB:A0A024RBG1",
  "term_label": "diphosphoinositol-polyphosphate diphosphatase activity",
  "gene_symbol": "NUDT4B"
}